trachea gland development [GO:0061153] (biological process) Relationships: is a type of GO:0048732; is part of GO:0061152 Definition: The progression of a trachea gland over time, from its formation to the mature structure. Trachea glands are found under the mucus of the trachea and secrete mucus, and agents that help protect the lung from injury and infection. Sources: GOC:dph